{
  "term_label": "plasma membrane",
  "gene_name": "Phospholipid scramblase 2",
  "term_id": "GO:0005886",
  "gene_symbol": "PLSCR2",
  "gene": "UniProtKB:Q9NRY7"
}